{
  "gene_symbol": "SHISA8",
  "term_label": "dendritic spine membrane",
  "gene_name": "Protein shisa-8",
  "gene": "UniProtKB:B8ZZ34",
  "term_id": "GO:0032591"
}